{
  "gene": "UniProtKB:Q0ZGT2",
  "term_id": "GO:0070593",
  "gene_name": "Nexilin",
  "term_label": "dendrite self-avoidance",
  "gene_symbol": "NEXN"
}